{
  "term_id": "GO:0009897",
  "gene": "UniProtKB:P32927",
  "gene_symbol": "CSF2RB",
  "term_label": "external side of plasma membrane",
  "gene_name": "Cytokine receptor common subunit beta"
}